granular vesicle [GO:1990005] (cellular component) Sources: NIF_Subcellular:sao478230652 Relationships: is a type of GO:0031410 Subtypes: neurosecretory vesicle [GO:1990008] Definition: A cytoplasmic membrane-bounded vesicle of varying size, but usually larger than 45 nm, with an electron dense granular core, found in noradrenergic and peptidergic cells.